{
  "gene": "UniProtKB:P14678",
  "gene_name": "Small nuclear ribonucleoprotein-associated proteins B and B'",
  "gene_symbol": "SNRPB",
  "term_label": "U2 snRNP",
  "term_id": "GO:0005686"
}